{
  "gene_name": "Transmembrane protein 178B",
  "term_label": "Unknown molecular function",
  "gene": "UniProtKB:H3BS89",
  "gene_symbol": "TMEM178B",
  "term_id": "UNKNOWN:0001"
}